regulation of protein localization to centrosome [GO:1904779] (biological process) Subtypes: GO:1904780, positive regulation of protein localization to centrosome [GO:1904781] Also known as: regulation of protein localisation to centrosome Definition: Any process that modulates the frequency, rate or extent of protein localization to centrosome. Note: An example is cdk-2 in C. elegans (UniProt ID O61847) in PMID:17115027 (inferred from mutant phenotype). Relationships: is a type of regulation of protein localization [GO:0032880]; regulates protein localization to centrosome [GO:0071539] References: PMID:17115027 Sources: GOC:TermGenie, GO_REF:0000058